{
  "gene_symbol": "NDUFA1",
  "gene_name": "NADH dehydrogenase [ubiquinone] 1 alpha subcomplex subunit 1",
  "term_id": "GO:0045271",
  "term_label": "respiratory chain complex I",
  "gene": "UniProtKB:O15239"
}